{
  "term_id": "GO:0003924",
  "gene": "UniProtKB:O00429",
  "gene_symbol": "DNM1L",
  "gene_name": "Dynamin-1-like protein",
  "term_label": "GTPase activity"
}